{
  "gene": "UniProtKB:A1L4L8",
  "term_label": "Unknown biological process",
  "gene_symbol": "PLAC8L1",
  "gene_name": "PLAC8-like protein 1",
  "term_id": "UNKNOWN:0002"
}